lateral cortical node assembly [GO:1903359] (biological process) Relationships: is a type of protein-containing complex assembly [GO:0065003] Definition: The aggregation, arrangement and bonding together of a set of components to form a lateral cortical node. Also known as: Skb1-containing cortical node assembly, Skb1-containing cortical node formation, lateral cortical node formation References: PMID:25009287 Sources: GOC:TermGenie, GO_REF:0000079